{
  "gene_symbol": "KMT5A",
  "term_id": "GO:0006357",
  "term_label": "regulation of transcription by RNA polymerase II",
  "gene_name": "N-lysine methyltransferase KMT5A",
  "gene": "UniProtKB:Q9NQR1"
}